{
  "term_label": "dendrite",
  "gene_symbol": "LRRK2",
  "term_id": "GO:0030425",
  "gene_name": "Leucine-rich repeat serine_threonine-protein kinase 2",
  "gene": "UniProtKB:Q5S007"
}